{
  "gene": "UniProtKB:Q3MJ40",
  "term_id": "UNKNOWN:0001",
  "gene_name": "Putative coiled-coil domain-containing protein 144B",
  "gene_symbol": "CCDC144BP",
  "term_label": "Unknown molecular function"
}